positive regulation of epithelial cell differentiation [GO:0030858] (biological process) Definition: Any process that activates or increases the frequency, rate or extent of epithelial cell differentiation. Relationships: is a type of regulation of epithelial cell differentiation [GO:0030856]; is a type of positive regulation of cell differentiation [GO:0045597]; positively regulates epithelial cell differentiation [GO:0030855] Also known as: up regulation of epithelial cell differentiation, up-regulation of epithelial cell differentiation, upregulation of epithelial cell differentiation, activation of epithelial cell differentiation, stimulation of epithelial cell differentiation Subtypes: positive regulation of polarized epithelial cell differentiation [GO:0030862], positive regulation of cumulus cell differentiation [GO:0045594], positive regulation of endothelial cell differentiation [GO:0045603], positive regulation of epidermal cell differentiation [GO:0045606], positive regulation of hepatocyte differentiation [GO:0070368], GO:1901248, positive regulation of lung goblet cell differentiation [GO:1901251], positive regulation of lens fiber cell differentiation [GO:1902748], GO:1902913, positive regulation of type B pancreatic cell development [GO:2000078], positive regulation of pancreatic A cell differentiation [GO:2000228], GO:2000698 Sources: GOC:mah